negative regulation of teliospore formation [GO:0075258] (biological process) Sources: GOC:pamgo_curators Relationships: is_a negative regulation of asexual sporulation resulting in formation of a cellular spore [GO:0043944]; is a type of GO:0075256; negatively regulates GO:0075255 Definition: Any process that stops, prevents, or reduces the frequency, rate or extent of teliospore formation, which is the formation of a thick-walled resting or overwintering spore produced by the rust fungi (Uredinales) and smut fungi (Ustilaginales) in which karyogamy occurs.